regulation of ethylene biosynthetic process [GO:0010364] (biological process) Definition: Any process that modulates the frequency, rate, or extent of an ethylene biosynthetic process. Sources: GOC:tair_curators Relationships: is a type of regulation of olefin biosynthetic process [GO:1900911]; regulates ethylene biosynthetic process [GO:0009693] Subtypes: GO:0010365, GO:0010366